{
  "gene": "UniProtKB:Q9NSP4",
  "term_label": "Unknown cellular component",
  "term_id": "UNKNOWN:0003",
  "gene_symbol": "CENPM",
  "gene_name": "Centromere protein M"
}